{
  "gene": "UniProtKB:O14598",
  "term_label": "Unknown molecular function",
  "term_id": "UNKNOWN:0001",
  "gene_symbol": "VCY",
  "gene_name": "Testis-specific basic protein Y 1"
}